demethylation [GO:0070988] (biological process) Definition: The process of removing one or more methyl groups from a molecule. Relationships: is a type of GO:0008152 Subtypes: protein demethylation [GO:0006482], oxidative demethylation [GO:0070989] Sources: GOC:BHF, GOC:rl